{
  "gene": "UniProtKB:Q6PRD1",
  "gene_symbol": "GPR179",
  "term_id": "UNKNOWN:0001",
  "gene_name": "Probable G-protein coupled receptor 179",
  "term_label": "Unknown molecular function"
}